{
  "gene_symbol": "ZNF415",
  "term_label": "RNA polymerase II cis-regulatory region sequence-specific DNA binding",
  "term_id": "GO:0000978",
  "gene_name": "Zinc finger protein 415",
  "gene": "UniProtKB:Q09FC8"
}